maintenance of vesicle location [GO:0051655] (biological process) Definition: Any process in which a vesicle is maintained in a specific location within a cell and prevented from moving elsewhere. Sources: GOC:ai, GOC:dph, GOC:tb Also known as: maintenance of vesicle localization Relationships: is a type of vesicle localization [GO:0051648]; is_a maintenance of organelle location [GO:0051657] Subtypes: maintenance of secretory granule location [GO:0032255], maintenance of pigment granule location [GO:0051906]